fucose binding [GO:0042806] (MF) Definition: Binding to fucose, the pentose 6-deoxygalactose. Sources: ISBN:0582227089 Relationships: is a type of monosaccharide binding [GO:0048029]